{
  "gene_symbol": "VSIG10L",
  "term_id": "UNKNOWN:0001",
  "gene": "UniProtKB:Q86VR7",
  "gene_name": "V-set and immunoglobulin domain-containing protein 10-like",
  "term_label": "Unknown molecular function"
}